D-xylose 1-dehydrogenase (NADP+) activity [GO:0047837] (MF) Definition: Catalysis of the reaction: D-xylose + NADP+ = D-xylono-1,5-lactone + H+ + NADPH. Also known as: D-xylose (nicotinamide adenine dinucleotide phosphate) dehydrogenase activity, D-xylose-NADP dehydrogenase activity, D-xylose:NADP+ 1-oxidoreductase activity, D-xylose:NADP+ oxidoreductase activity Relationships: is_a oxidoreductase activity, acting on the CH-OH group of donors, NAD or NADP as acceptor [GO:0016616] Sources: RHEA:22000